transduction [GO:0009293] (biological process) Definition: A type of horizontal gene transfer in which genetic material is introduced into a cell mediated by a virus. Note: This process occurs both in prokaryotes and in eukaryotes. Relationships: is_a horizontal gene transfer [GO:0009292] References: PMID:18265289, PMID:33597173